bile acid binding [GO:0032052] (molecular function) Relationships: is a type of GO:0033293 Sources: GOC:rph Definition: Binding to a bile acid, a steroid carboxylic acids occurring in bile. Subtypes: lithocholic acid binding [GO:1902121], GO:1902122